{
  "gene_name": "Synaptotagmin-like protein 1",
  "gene_symbol": "SYTL1",
  "term_label": "plasma membrane",
  "gene": "UniProtKB:Q8IYJ3",
  "term_id": "GO:0005886"
}